{
  "term_id": "GO:0035371",
  "gene": "UniProtKB:Q9Y448",
  "gene_name": "Small kinetochore-associated protein",
  "gene_symbol": "KNSTRN",
  "term_label": "microtubule plus-end"
}